{
  "gene_name": "Rabphilin-3A",
  "term_id": "GO:0098850",
  "gene_symbol": "RPH3A",
  "gene": "UniProtKB:Q9Y2J0",
  "term_label": "extrinsic component of synaptic vesicle membrane"
}